{
  "term_id": "GO:0030317",
  "gene": "UniProtKB:Q7RTX7",
  "term_label": "flagellated sperm motility",
  "gene_name": "Cation channel sperm-associated protein 4",
  "gene_symbol": "CATSPER4"
}